{
  "term_id": "GO:0016323",
  "term_label": "basolateral plasma membrane",
  "gene_symbol": "DLG1",
  "gene_name": "Disks large homolog 1",
  "gene": "UniProtKB:Q12959"
}